{
  "term_label": "Unknown molecular function",
  "gene_symbol": "DAAM2",
  "term_id": "UNKNOWN:0001",
  "gene": "UniProtKB:Q86T65",
  "gene_name": "Disheveled-associated activator of morphogenesis 2"
}